{
  "term_label": "DNA-binding transcription factor activity, RNA polymerase II-specific",
  "gene_symbol": "ZNF557",
  "term_id": "GO:0000981",
  "gene_name": "Zinc finger protein 557",
  "gene": "UniProtKB:Q8N988"
}